cellular response to iron(II) ion [GO:0071282] (biological process) Definition: Any process that results in a change in state or activity of a cell (in terms of movement, secretion, enzyme production, gene expression, etc.) as a result of an iron(II) ion stimulus. Sources: GOC:mah Also known as: cellular response to iron(II) Relationships: is a type of response to iron(II) ion [GO:0010040]; is_a GO:0071281